{
  "gene_name": "Z-DNA-binding protein 1",
  "gene_symbol": "ZBP1",
  "term_label": "positive regulation of apoptotic process",
  "term_id": "GO:0043065",
  "gene": "UniProtKB:Q9H171"
}